{
  "term_label": "Unknown biological process",
  "term_id": "UNKNOWN:0002",
  "gene": "UniProtKB:Q8IZU2",
  "gene_name": "WD repeat-containing protein 17",
  "gene_symbol": "WDR17"
}